positive regulation of prolactin signaling pathway [GO:1902213] (biological process) Definition: Any process that activates or increases the frequency, rate or extent of prolactin signaling pathway. Relationships: is a type of positive regulation of cytokine-mediated signaling pathway [GO:0001961]; is_a regulation of prolactin signaling pathway [GO:1902211]; positively regulates prolactin signaling pathway [GO:0038161] References: PMID:11773439 Sources: GOC:TermGenie Also known as: positive regulation of PRL signaling pathway, positive regulation of prolactin-mediated signaling pathway, up regulation of PRL signaling pathway, up regulation of prolactin signaling pathway, up regulation of prolactin-mediated signaling pathway, up-regulation of PRL signaling pathway, up-regulation of prolactin signaling pathway, up-regulation of prolactin-mediated signaling pathway, upregulation of PRL signaling pathway, upregulation of prolactin signaling pathway, upregulation of prolactin-mediated signaling pathway, activation of PRL signaling pathway, activation of prolactin signaling pathway, activation of prolactin-mediated signaling pathway